mannan exo-1,2-1,6-alpha-mannosidase activity [GO:0033941] (molecular function) Also known as: 1,2-1,6-alpha-D-mannan D-mannohydrolase activity, exo-1,2-1,6-alpha-mannosidase activity Relationships: is a type of alpha-mannosidase activity [GO:0004559] Definition: Catalysis of the hydrolysis of (1->2)-alpha-D- and (1->6)-alpha-D- linkages in mannan, releasing D-mannose. Sources: EC:3.2.1.137